sperm aster formation [GO:0035044] (biological process) Sources: GOC:bf, ISBN:0879694238 Definition: Formation and organization of an aster composed of microtubule arrays originating from the sperm basal body and extending virtually to the egg periphery. The sperm aster ensures the appropriate positioning of the male and female pronuclei. Relationships: is a type of microtubule cytoskeleton organization [GO:0000226]; is part of single fertilization [GO:0007338]